{
  "gene": "UniProtKB:Q8TAA1",
  "gene_symbol": "RNASE11",
  "term_id": "UNKNOWN:0003",
  "term_label": "Unknown cellular component",
  "gene_name": "Probable ribonuclease 11"
}